{
  "gene": "UniProtKB:Q5VU69",
  "gene_symbol": "CFAP141",
  "term_label": "Unknown cellular component",
  "gene_name": "Cilia- and flagella-associated protein 141",
  "term_id": "UNKNOWN:0003"
}